{
  "term_label": "RNA polymerase II cis-regulatory region sequence-specific DNA binding",
  "gene_name": "MAX gene-associated protein",
  "gene": "UniProtKB:Q8IWI9",
  "gene_symbol": "MGA",
  "term_id": "GO:0000978"
}